{
  "term_label": "cytoplasm",
  "gene_name": "PRAME family member 14",
  "term_id": "GO:0005737",
  "gene": "UniProtKB:Q5SWL7",
  "gene_symbol": "PRAMEF14"
}